{
  "gene": "UniProtKB:Q9UKF2",
  "term_label": "sperm head plasma membrane",
  "term_id": "GO:1990913",
  "gene_symbol": "ADAM30",
  "gene_name": "Disintegrin and metalloproteinase domain-containing protein 30"
}